{
  "term_id": "GO:0043514",
  "gene_name": "Interleukin-12 subunit beta",
  "gene_symbol": "IL12B",
  "term_label": "interleukin-12 complex",
  "gene": "UniProtKB:P29460"
}